{
  "gene": "UniProtKB:P52333",
  "gene_name": "Tyrosine-protein kinase JAK3",
  "gene_symbol": "JAK3",
  "term_label": "intracellular signal transduction",
  "term_id": "GO:0035556"
}